{
  "term_label": "Unknown biological process",
  "gene_name": "Solute carrier family 35 member F6",
  "term_id": "UNKNOWN:0002",
  "gene": "UniProtKB:Q8N357",
  "gene_symbol": "SLC35F6"
}